{
  "gene": "UniProtKB:Q495Y8",
  "gene_symbol": "SPDYE2",
  "term_id": "UNKNOWN:0002",
  "term_label": "Unknown biological process",
  "gene_name": "Speedy protein E2"
}